{
  "gene": "UniProtKB:Q9BY43",
  "gene_symbol": "CHMP4A",
  "term_id": "GO:0000815",
  "term_label": "ESCRT III complex",
  "gene_name": "Charged multivesicular body protein 4a"
}